{
  "gene_symbol": "CADM1",
  "term_id": "GO:0005102",
  "gene": "UniProtKB:Q9BY67",
  "term_label": "signaling receptor binding",
  "gene_name": "Cell adhesion molecule 1"
}